{
  "gene_name": "C-X-C motif chemokine 17",
  "gene_symbol": "CXCL17",
  "term_id": "GO:0010759",
  "gene": "UniProtKB:Q6UXB2",
  "term_label": "positive regulation of macrophage chemotaxis"
}